C-X-C chemokine receptor activity [GO:0016494] (molecular function) Subtypes: GO:0004918, C-X-C motif chemokine 12 receptor activity [GO:0038147] Definition: Combining with a C-X-C chemokine and transmitting the signal from one side of the membrane to the other to initiate a change in cell activity. A C-X-C chemokine has a single amino acid between the first two cysteines of the characteristic four cysteine motif. Relationships: is a type of chemokine receptor activity [GO:0004950]; has part C-X-C chemokine binding [GO:0019958] References: PMID:8662823 Sources: GOC:signaling